{
  "term_id": "GO:0046651",
  "gene_symbol": "HELLS",
  "gene": "UniProtKB:Q9NRZ9",
  "term_label": "lymphocyte proliferation",
  "gene_name": "Lymphoid-specific helicase"
}